nickel cation transmembrane transporter activity [GO:0015099] (molecular function) Subtypes: ABC-type nickel transporter activity [GO:0015413], high-affinity nickel cation transmembrane transporter activity [GO:0044750] Definition: Enables the transfer of nickel (Ni) cations from one side of a membrane to the other. Relationships: is a type of transition metal ion transmembrane transporter activity [GO:0046915]; BFO_0000050 GO:0035444 Also known as: zinc, cadmium, cobalt, nickel, lead-efflux ATPase activity Sources: GOC:ai